pyridoxine 4-oxidase activity [GO:0050237] (molecular function) Sources: EC:1.1.3.12, MetaCyc:PYRIDOXINE-4-OXIDASE-RXN Relationships: is a type of GO:0016899 Also known as: pyridoxin 4-oxidase activity, pyridoxine:oxygen 4-oxidoreductase activity, pyridoxol 4-oxidase activity Definition: Catalysis of the reaction: pyridoxine + O2 = pyridoxal + H2O2.